{
  "term_label": "collagen binding",
  "gene_symbol": "PCOLCE2",
  "gene_name": "Procollagen C-endopeptidase enhancer 2",
  "term_id": "GO:0005518",
  "gene": "UniProtKB:Q9UKZ9"
}